{
  "gene": "UniProtKB:A0A6I8PU40",
  "term_label": "Unknown cellular component",
  "gene_symbol": "TUG1",
  "gene_name": "Taurine up-regulated 1 protein",
  "term_id": "UNKNOWN:0003"
}